scopolamine biosynthetic process [GO:1900991] (biological process) Definition: The chemical reactions and pathways resulting in the formation of scopolamine. Relationships: is a type of GO:0009710; is a type of epoxide metabolic process [GO:0097176]; is a type of ether biosynthetic process [GO:1901503] References: PMID:16720272, PMID:18251710, PMID:32879484 Sources: GOC:TermGenie, GOC:yaf Also known as: scopolamine metabolic process, scopolamine metabolism, scopolamine anabolism, scopolamine biosynthesis, scopolamine formation, scopolamine synthesis